{
  "term_id": "UNKNOWN:0002",
  "gene": "UniProtKB:Q6ZUT9",
  "term_label": "Unknown biological process",
  "gene_symbol": "DENND5B",
  "gene_name": "DENN domain-containing protein 5B"
}